{
  "term_label": "nucleus",
  "gene_name": "Zinc finger protein 37A",
  "gene": "UniProtKB:P17032",
  "term_id": "GO:0005634",
  "gene_symbol": "ZNF37A"
}